{
  "term_id": "GO:0070971",
  "term_label": "endoplasmic reticulum exit site",
  "gene_symbol": "CTAGE6",
  "gene_name": "cTAGE family member 6",
  "gene": "UniProtKB:Q86UF2"
}